protein O-linked glycosylation via glucose [GO:0180059] (BP) Also known as: protein O-linked glucosylation Definition: A glycoprotein biosynthetic process starting with the covalent linkage of a glucose via a beta-glycosidic bond to the oxygen atom of a serine, threonine or tyrosine side chain in a protein, which can be further elongated with the sequential addition of sugar units resulting in the formation of a protein O-linked glycan. Relationships: is a type of protein O-linked glycosylation [GO:0006493] References: PMID:35536928